{
  "gene": "UniProtKB:Q8N5Y2",
  "gene_name": "Male-specific lethal 3 homolog",
  "term_label": "Unknown molecular function",
  "term_id": "UNKNOWN:0001",
  "gene_symbol": "MSL3"
}